{
  "gene": "UniProtKB:P22301",
  "gene_symbol": "IL10",
  "term_id": "GO:0050728",
  "gene_name": "Interleukin-10",
  "term_label": "negative regulation of inflammatory response"
}